{
  "gene_symbol": "IL1B",
  "gene": "UniProtKB:P01584",
  "gene_name": "Interleukin-1 beta",
  "term_label": "positive regulation of canonical NF-kappaB signal transduction",
  "term_id": "GO:0043123"
}